depsipeptide biosynthetic process [GO:0050763] (biological process) Subtypes: enniatin biosynthetic process [GO:0046585], emericellamide biosynthetic process [GO:1900557] Also known as: depsipeptide anabolism, depsipeptide biosynthesis, depsipeptide formation, depsipeptide synthesis Relationships: is a type of amide biosynthetic process [GO:0043604]; is a type of GO:0050761 Definition: The chemical reactions and pathways resulting in the formation of depsipeptides, a linear or cyclic compound composed of both amino acids and hydroxy acids in peptide and ester bonds respectively. Sources: GOC:go_curators